{
  "gene_symbol": "URGCP",
  "term_label": "Unknown cellular component",
  "gene": "UniProtKB:Q8TCY9",
  "gene_name": "Up-regulator of cell proliferation",
  "term_id": "UNKNOWN:0003"
}